{
  "term_label": "Unknown cellular component",
  "term_id": "UNKNOWN:0003",
  "gene": "UniProtKB:Q7M4L6",
  "gene_symbol": "SHF",
  "gene_name": "SH2 domain-containing adapter protein F"
}